{
  "term_id": "GO:0005615",
  "gene_symbol": "CCN2",
  "term_label": "extracellular space",
  "gene": "UniProtKB:P29279",
  "gene_name": "CCN family member 2"
}